{
  "term_label": "plasma membrane",
  "term_id": "GO:0005886",
  "gene_name": "Basal cell adhesion molecule",
  "gene": "UniProtKB:P50895",
  "gene_symbol": "BCAM"
}